leukotriene receptor activity [GO:0004974] (molecular function) Definition: Combining with a leukotriene to initiate a change in cell activity. Leukotrienes are pharmacologically active substances with a set of three conjugated double bonds; some contain a peptide group based on cysteine. Subtypes: cysteinyl leukotriene receptor activity [GO:0001631], leukotriene B4 receptor activity [GO:0001632] Relationships: is a type of GO:0004953; is part of leukotriene signaling pathway [GO:0061737] Sources: GOC:ai, ISBN:0198506732